positive regulation of response to propan-1-ol [GO:1901447] (biological process) Relationships: is a type of positive regulation of response to alcohol [GO:1901421]; is a type of regulation of response to propan-1-ol [GO:1901445]; positively regulates response to propan-1-ol [GO:1901427] Sources: GOC:TermGenie, GOC:mengo_curators Definition: Any process that activates or increases the frequency, rate or extent of response to propan-1-ol. Also known as: up regulation of response to propan-1-ol, up-regulation of response to propan-1-ol, upregulation of response to propan-1-ol, activation of response to propan-1-ol